{
  "gene_name": "Leucine-rich repeat-containing protein 52",
  "term_id": "GO:0099104",
  "gene_symbol": "LRRC52",
  "term_label": "potassium channel activator activity",
  "gene": "UniProtKB:Q8N7C0"
}